{
  "gene": "UniProtKB:P40818",
  "term_id": "GO:0007032",
  "gene_name": "Ubiquitin carboxyl-terminal hydrolase 8",
  "term_label": "endosome organization",
  "gene_symbol": "USP8"
}